{
  "gene_symbol": "PPP1R15A",
  "gene_name": "Protein phosphatase 1 regulatory subunit 15A",
  "gene": "UniProtKB:O75807",
  "term_id": "GO:0005783",
  "term_label": "endoplasmic reticulum"
}